{
  "gene_symbol": "ZNF621",
  "term_id": "GO:0000978",
  "term_label": "RNA polymerase II cis-regulatory region sequence-specific DNA binding",
  "gene_name": "Zinc finger protein 621",
  "gene": "UniProtKB:Q6ZSS3"
}